{
  "gene_name": "Protein preY, mitochondrial",
  "term_id": "UNKNOWN:0001",
  "term_label": "Unknown molecular function",
  "gene": "UniProtKB:Q96I23",
  "gene_symbol": "PYURF"
}